{
  "gene_symbol": "TEDC1",
  "term_id": "UNKNOWN:0001",
  "gene": "UniProtKB:Q86SX3",
  "term_label": "Unknown molecular function",
  "gene_name": "Tubulin epsilon and delta complex protein 1"
}